{
  "term_label": "Unknown biological process",
  "gene_symbol": "OR5A2",
  "term_id": "UNKNOWN:0002",
  "gene_name": "Olfactory receptor 5A2",
  "gene": "UniProtKB:Q8NGI9"
}